{
  "gene_name": "Syntaxin-11",
  "gene": "UniProtKB:O75558",
  "term_id": "GO:0006886",
  "gene_symbol": "STX11",
  "term_label": "intracellular protein transport"
}